{
  "term_label": "Unknown biological process",
  "term_id": "UNKNOWN:0002",
  "gene_name": "Tetratricopeptide repeat protein 9B",
  "gene": "UniProtKB:Q8N6N2",
  "gene_symbol": "TTC9B"
}